{
  "gene": "UniProtKB:Q9NXB9",
  "term_id": "GO:0009922",
  "gene_name": "Elongation of very long chain fatty acids protein 2",
  "term_label": "fatty acid elongase activity",
  "gene_symbol": "ELOVL2"
}